folic acid metabolic process [GO:0046655] (BP) Definition: The chemical reactions and pathways involving folic acid, pteroylglutamic acid. Folic acid is widely distributed as a member of the vitamin B complex and is essential for the synthesis of purine and pyrimidines. Sources: ISBN:0198506732 Also known as: folate metabolic process, folate metabolism, folic acid metabolism, vitamin B9 metabolic process, vitamin B9 metabolism, vitamin M metabolic process, vitamin M metabolism Subtypes: GO:0046656, folic acid catabolic process [GO:0046657] Relationships: is a type of folic acid-containing compound metabolic process [GO:0006760]; is_a amide metabolic process [GO:0043603]; is a type of dicarboxylic acid metabolic process [GO:0043648]